positive regulation of protein-containing complex assembly [GO:0031334] (biological process) Definition: Any process that activates or increases the frequency, rate or extent of protein complex assembly. Sources: GOC:mah Subtypes: positive regulation of exocyst assembly [GO:0001930], GO:0006293, positive regulation of synaptic vesicle priming [GO:0010808], positive regulation of protein polymerization [GO:0032273], positive regulation of protein oligomerization [GO:0032461], GO:0033625, positive regulation of SNARE complex assembly [GO:0035543], positive regulation of RNA polymerase II transcription preinitiation complex assembly [GO:0045899], GO:0062165, positive regulation of podosome assembly [GO:0071803], GO:0090035, GO:0090108, GO:0140887, positive regulation of AIM2 inflammasome complex assembly [GO:0140973], positive regulation of NLRP3 inflammasome complex assembly [GO:1900227], GO:1900514, GO:1901192, positive regulation of formation of translation preinitiation complex [GO:1901195], positive regulation of assembly of large subunit precursor of preribosome [GO:1902628], positive regulation of VCP-NPL4-UFD1 AAA ATPase complex assembly [GO:1904241], positive regulation of Wnt-Frizzled-LRP5/6 complex assembly [GO:1904712], positive regulation of shelterin complex assembly [GO:1904792], positive regulation of beta-catenin-TCF complex assembly [GO:1904865], positive regulation of telomerase catalytic core complex assembly [GO:1904884], positive regulation of apoptosome assembly [GO:1905102], positive regulation of clathrin coat assembly [GO:1905445], GO:1905511, positive regulation of eukaryotic translation initiation factor 4F complex assembly [GO:1905537], positive regulation of kinetochore assembly [GO:1905561], positive regulation of FACT complex assembly [GO:1905646], positive regulation of Atg1/ULK1 kinase complex assembly [GO:1905866], positive regulation of mediator complex assembly [GO:2001178] Also known as: up regulation of protein complex assembly, up-regulation of protein complex assembly, upregulation of protein complex assembly, activation of protein complex assembly, stimulation of protein complex assembly, positive regulation of protein complex assembly Relationships: is a type of regulation of protein-containing complex assembly [GO:0043254]; is a type of positive regulation of cellular component biogenesis [GO:0044089]; is_a GO:0051130; positively regulates protein-containing complex assembly [GO:0065003]